complement activation [GO:0006956] (biological process) Also known as: complement cascade, complement response, complement activity Relationships: is a type of immune effector process [GO:0002252]; is a type of GO:0002253; is a type of GO:0006959; has part protein activation cascade [GO:0072376] Sources: GOC:add, GO_REF:0000022, ISBN:0781735149 Regulation: regulated by regulation of complement activation [GO:0030449]; negatively regulated by negative regulation of complement activation [GO:0045916]; positively regulated by positive regulation of complement activation [GO:0045917] Definition: Any process involved in the activation of any of the steps of the complement cascade, which allows for the direct killing of microbes, the disposal of immune complexes, and the regulation of other immune processes; the initial steps of complement activation involve one of three pathways, the classical pathway, the alternative pathway, and the lectin pathway, all of which lead to the terminal complement pathway. Subtypes: complement activation, lectin pathway [GO:0001867], activation of membrane attack complex [GO:0001905], complement activation, alternative pathway [GO:0006957], complement activation, classical pathway [GO:0006958], complement activation, GZMK pathway [GO:0160257]